{
  "term_id": "GO:0005764",
  "gene_symbol": "ELAPOR1",
  "gene": "UniProtKB:Q6UXG2",
  "term_label": "lysosome",
  "gene_name": "Endosome_lysosome-associated apoptosis and autophagy regulator 1"
}